{
  "term_label": "nucleus",
  "gene_name": "Nuclear factor of activated T-cells, cytoplasmic 3",
  "term_id": "GO:0005634",
  "gene_symbol": "NFATC3",
  "gene": "UniProtKB:Q12968"
}